{
  "term_label": "glyoxal metabolic process",
  "gene_symbol": "PARK7",
  "gene": "UniProtKB:Q99497",
  "gene_name": "Parkinson disease protein 7",
  "term_id": "GO:1903189"
}